cellular response to astaxanthin [GO:1905218] (biological process) Definition: Any process that results in a change in state or activity of a cell (in terms of movement, secretion, enzyme production, gene expression, etc.) as a result of an astaxanthin stimulus. References: PMID:22309505 Sources: GOC:TermGenie, GO_REF:0000071 Also known as: cellular response to (3S,3'S)-3,3'-dihydroxy-beta,beta-carotene-4,4'-dione Relationships: is a type of GO:0071396; is_a response to astaxanthin [GO:1905217]